{
  "term_id": "GO:1990904",
  "gene_symbol": "PABPC1L2A",
  "term_label": "ribonucleoprotein complex",
  "gene_name": "Polyadenylate-binding protein 1-like 2",
  "gene": "UniProtKB:Q5JQF8"
}